{
  "gene": "UniProtKB:A0A494C191",
  "term_id": "GO:0019901",
  "term_label": "protein kinase binding",
  "gene_symbol": "SPDYE9",
  "gene_name": "Putative speedy protein E9"
}